{
  "term_id": "GO:0042981",
  "gene_name": "Ubiquitin carboxyl-terminal hydrolase 17-like protein 6",
  "term_label": "regulation of apoptotic process",
  "gene_symbol": "USP17L6P",
  "gene": "UniProtKB:Q6QN14"
}